mating pheromone secretion [GO:0071834] (BP) Relationships: is a type of peptide hormone secretion [GO:0030072] Sources: GOC:mah Definition: The regulated release of a mating pheromone, a peptide hormone that induces a behavioral or physiological response(s) from a responding organism or cell, that contributes to a process of sexual reproduction. Also known as: mating-type pheromone secretion Subtypes: GO:0071631, mating pheromone secretion involved in regulation of conjugation with cellular fusion [GO:0071835]